{
  "term_id": "GO:0006357",
  "gene": "UniProtKB:O75820",
  "gene_symbol": "ZNF189",
  "gene_name": "Zinc finger protein 189",
  "term_label": "regulation of transcription by RNA polymerase II"
}